endothelial cell-matrix adhesion [GO:0090673] (biological process) References: PMID:19460962 Sources: GOC:BHF, GOC:BHF_miRNA, GOC:bc Definition: The binding of an endothelial cell to the extracellular matrix via adhesion molecules. Relationships: is a type of cell-matrix adhesion [GO:0007160] Regulation: regulated by regulation of endothelial cell-matrix adhesion [GO:1904904]; negatively regulated by negative regulation of endothelial cell-matrix adhesion [GO:1904905]; positively regulated by positive regulation of endothelial cell-matrix adhesion [GO:1904906]